{
  "term_id": "GO:0008107",
  "gene": "UniProtKB:P19526",
  "term_label": "galactoside 2-alpha-L-fucosyltransferase activity",
  "gene_name": "Galactoside alpha-(1,2)-fucosyltransferase 1",
  "gene_symbol": "FUT1"
}